{
  "term_label": "Unknown biological process",
  "term_id": "UNKNOWN:0002",
  "gene_symbol": "MRPS18B",
  "gene_name": "Small ribosomal subunit protein mS40",
  "gene": "UniProtKB:Q9Y676"
}